{
  "gene": "UniProtKB:Q5MJ68",
  "term_id": "UNKNOWN:0002",
  "gene_name": "Speedy protein C",
  "gene_symbol": "SPDYC",
  "term_label": "Unknown biological process"
}